regulation of actomyosin contractile ring contraction [GO:0031991] (biological process) Definition: Any process that modulates the frequency, rate or extent of contraction of the actomyosin ring involved in cytokinesis that takes place as part of a cell cycle. Sources: GOC:dph, GOC:mah, GOC:tb Also known as: regulation of actomyosin contractile ring constriction, regulation of contractile ring contraction involved in cell cycle cytokinesis, regulation of contractile ring contraction involved in cytokinesis during cell cycle Relationships: is a type of cytokinetic process [GO:0032506]; is a type of regulation of cytokinetic process [GO:0032954]; regulates actomyosin contractile ring contraction [GO:0000916] Subtypes: GO:1903471